3-(hydroxyamino)phenol mutase activity [GO:0034022] (molecular function) Sources: EC:5.4.4.3, RHEA:20577 Relationships: is a type of intramolecular hydroxytransferase activity [GO:0050486] Also known as: 3-(hydroxyamino)phenol hydroxymutase activity, 3-hydroxylaminophenol mutase activity, 3HAP mutase activity Definition: Catalysis of the reaction: 3-hydroxyaminophenol = aminohydroquinone.